{
  "term_label": "DNA-binding transcription factor activity, RNA polymerase II-specific",
  "gene": "UniProtKB:Q12948",
  "gene_name": "Forkhead box protein C1",
  "term_id": "GO:0000981",
  "gene_symbol": "FOXC1"
}